{
  "gene_symbol": "KRT12",
  "gene": "UniProtKB:Q99456",
  "gene_name": "Keratin, type I cytoskeletal 12",
  "term_label": "keratin filament",
  "term_id": "GO:0045095"
}